{
  "gene_symbol": "DNAJB2",
  "term_label": "cytosol",
  "gene": "UniProtKB:P25686",
  "gene_name": "DnaJ homolog subfamily B member 2",
  "term_id": "GO:0005829"
}